{
  "gene_name": "EH domain-containing protein 4",
  "term_id": "GO:0030674",
  "gene_symbol": "EHD4",
  "term_label": "protein-macromolecule adaptor activity",
  "gene": "UniProtKB:Q9H223"
}